{
  "gene_name": "Kelch-like protein 23",
  "gene": "UniProtKB:Q8NBE8",
  "term_label": "Cul3-RING ubiquitin ligase complex",
  "gene_symbol": "KLHL23",
  "term_id": "GO:0031463"
}